{
  "gene": "UniProtKB:P49662",
  "term_label": "Unknown molecular function",
  "gene_symbol": "CASP4",
  "gene_name": "Caspase-4",
  "term_id": "UNKNOWN:0001"
}